{
  "gene_symbol": "LNP1",
  "term_label": "Unknown cellular component",
  "gene_name": "Leukemia NUP98 fusion partner 1",
  "term_id": "UNKNOWN:0003",
  "gene": "UniProtKB:A1A4G5"
}